{
  "gene": "UniProtKB:Q15599",
  "term_label": "apical plasma membrane",
  "term_id": "GO:0016324",
  "gene_name": "Na(+)_H(+) exchange regulatory cofactor NHE-RF2",
  "gene_symbol": "NHERF2"
}